{
  "gene": "UniProtKB:P16401",
  "term_label": "nucleosomal DNA binding",
  "gene_symbol": "H1-5",
  "gene_name": "Histone H1.5",
  "term_id": "GO:0031492"
}